{
  "gene": "UniProtKB:Q9HAN9",
  "gene_name": "Nicotinamide_nicotinic acid mononucleotide adenylyltransferase 1",
  "term_id": "GO:0034355",
  "term_label": "NAD+ biosynthetic process via the salvage pathway",
  "gene_symbol": "NMNAT1"
}